{
  "gene": "UniProtKB:Q9BUA3",
  "gene_symbol": "SPINDOC",
  "term_label": "Unknown cellular component",
  "gene_name": "Spindlin interactor and repressor of chromatin-binding protein",
  "term_id": "UNKNOWN:0003"
}